pentose biosynthetic process [GO:0019322] (biological process) Definition: The chemical reactions and pathways resulting in the formation of a pentose, any monosaccharide with a chain of five carbon atoms in the molecule. Sources: ISBN:0198506732 Also known as: pentose anabolism, pentose biosynthesis, pentose formation, pentose synthesis Relationships: is a type of pentose metabolic process [GO:0019321]; is a type of monosaccharide biosynthetic process [GO:0046364] Subtypes: xylulose biosynthetic process [GO:0005999], D-ribose biosynthetic process [GO:0019302], GO:0019567, GO:0042842